cresol catabolic process [GO:0046199] (biological process) Definition: The chemical reactions and pathways resulting in the breakdown of cresol, a mixture of the aromatic alcohol isoforms o-, p-, and m-cresol, which is obtained from coal tar or petroleum. The isomers are used as disinfectants, textile scouring agents, surfactants and as intermediates in the manufacture of salicylaldehyde, coumarin, and herbicides as well as being a major component of creosote. Sources: GOC:ai Also known as: cresol breakdown, cresol catabolism, cresol degradation Relationships: is a type of GO:0019336; is a type of xenobiotic catabolic process [GO:0042178]; is a type of toluene-containing compound catabolic process [GO:0072491] Subtypes: GO:0042213, p-cresol catabolic process [GO:1901785]